{
  "term_id": "GO:0000467",
  "gene": "UniProtKB:Q15024",
  "term_label": "exonucleolytic trimming to generate mature 3'-end of 5.8S rRNA from tricistronic rRNA transcript (SSU-rRNA, 5.8S rRNA, LSU-rRNA)",
  "gene_symbol": "EXOSC7",
  "gene_name": "Exosome complex component RRP42"
}